{
  "gene": "UniProtKB:Q8N138",
  "gene_symbol": "ORMDL3",
  "term_id": "UNKNOWN:0001",
  "gene_name": "ORM1-like protein 3",
  "term_label": "Unknown molecular function"
}